{
  "term_id": "GO:0050911",
  "gene": "UniProtKB:Q9H207",
  "gene_name": "Olfactory receptor 10A5",
  "term_label": "detection of chemical stimulus involved in sensory perception of smell",
  "gene_symbol": "OR10A5"
}